{
  "gene": "UniProtKB:Q6NZY7",
  "gene_name": "Cdc42 effector protein 5",
  "term_label": "small GTPase binding",
  "term_id": "GO:0031267",
  "gene_symbol": "CDC42EP5"
}